lens fiber cell development [GO:0070307] (biological process) Definition: The process whose specific outcome is the progression of a lens fiber cell over time, from its formation to the mature structure. Cell development does not include the steps involved in committing a cell to a lens fiber cell fate. A lens fiber cell is any of the elongated, tightly packed cells that make up the bulk of the mature lens in a camera-type eye. References: PMID:7693735 Sources: GOC:mah Relationships: is a type of epithelial cell development [GO:0002064]; is part of GO:0070306 Also known as: lens fibre cell development